2'-(5''-triphosphoribosyl)-3'-dephospho-CoA biosynthetic process [GO:0019361] (biological process) Sources: GOC:ai Also known as: 2'-(5''-triphosphoribosyl)-3'-dephospho-CoA anabolism, 2'-(5''-triphosphoribosyl)-3'-dephospho-CoA biosynthesis, 2'-(5''-triphosphoribosyl)-3'-dephospho-CoA formation, 2'-(5''-triphosphoribosyl)-3'-dephospho-CoA synthesis Relationships: is_a GO:0009152 Definition: The chemical reactions and pathways resulting in the formation of 2'-(5''-triphosphoribosyl)-3'-dephospho-CoA, a derivative of coenzyme A.